positive regulation of neuron projection regeneration [GO:0070572] (biological process) Definition: Any process that activates or increases the frequency, rate or extent of neuron projection regeneration, the regrowth of neuronal processes such as axons or dendrites following their loss or damage. Subtypes: positive regulation of axon regeneration [GO:0048680] Relationships: is a type of positive regulation of neuron projection development [GO:0010976]; is a type of positive regulation of response to stimulus [GO:0048584]; is a type of positive regulation of developmental process [GO:0051094]; is a type of regulation of neuron projection regeneration [GO:0070570]; positively regulates neuron projection regeneration [GO:0031102] Sources: GOC:mah